{
  "term_id": "GO:0005789",
  "gene_symbol": "JPH1",
  "gene": "UniProtKB:Q9HDC5",
  "term_label": "endoplasmic reticulum membrane",
  "gene_name": "Junctophilin-1"
}